diuretic hormone activity [GO:0008613] (molecular function) Relationships: is a type of GO:0005179 Definition: The action characteristic of a diuretic hormone, a peptide hormone that, upon receptor binding, regulates water balance and fluid secretion. References: PMID:8618894 Sources: GOC:mah, InterPro:IPR003621